female somatic sex determination [GO:0019101] (biological process) Definition: The determination of sex and sexual phenotypes in a female organism's soma. Relationships: is a type of GO:0018993; is a type of GO:0030237 Sources: GOC:mah